male-specific defense response to bacterium [GO:0050831] (biological process) Also known as: male-specific defence response to bacteria, male-specific defence response to bacterium, male-specific defense response to bacteria, male-specific antibacterial peptide activity Definition: A set of reactions, specific to males, that are triggered in response to the presence of a bacterium that act to protect the cell or organism. Relationships: is a type of GO:0042742 Sources: GOC:ai Subtypes: male-specific antibacterial humoral response [GO:0006962]